ethanolamine transport [GO:0034229] (biological process) Definition: The directed movement of ethanolamine into, out of or within a cell, or between cells, by means of some agent such as a transporter or pore. Ethanolamine (2-aminoethanol, monoethanolamine) is an amino alcohol that occurs widely in living organisms as a constituent of certain types of phospholipids, such as phosphatidylethanolamine. Relationships: is a type of GO:0015695; is a type of amine transport [GO:0015837]; is_a organic hydroxy compound transport [GO:0015850] References: PMID:3514579 Sources: GOC:rn Also known as: 2-aminoethanol transport, monoethanolamine transport